{
  "gene": "UniProtKB:Q86XD8",
  "term_label": "Unknown cellular component",
  "term_id": "UNKNOWN:0003",
  "gene_name": "AN1-type zinc finger protein 4",
  "gene_symbol": "ZFAND4"
}